{
  "gene_symbol": "ENY2",
  "term_id": "GO:0006357",
  "gene": "UniProtKB:Q9NPA8",
  "term_label": "regulation of transcription by RNA polymerase II",
  "gene_name": "Transcription and mRNA export factor ENY2"
}